{
  "gene_symbol": "FAM157C",
  "term_label": "Unknown molecular function",
  "gene_name": "Putative protein FAM157C",
  "term_id": "UNKNOWN:0001",
  "gene": "UniProtKB:P0CG43"
}